{
  "term_id": "UNKNOWN:0003",
  "term_label": "Unknown cellular component",
  "gene_name": "Putative uncharacterized protein FLJ46204",
  "gene": "UniProtKB:Q6ZRP5",
  "gene_symbol": "Q6ZRP5"
}